{
  "term_label": "superoxide-generating NADPH oxidase activator activity",
  "term_id": "GO:0016176",
  "gene_symbol": "SH3PXD2B",
  "gene": "UniProtKB:A1X283",
  "gene_name": "SH3 and PX domain-containing protein 2B"
}